{
  "term_label": "negative regulation of transcription by RNA polymerase II",
  "gene_name": "E3 SUMO-protein ligase CBX4",
  "gene_symbol": "CBX4",
  "term_id": "GO:0000122",
  "gene": "UniProtKB:O00257"
}